{
  "gene": "UniProtKB:P48061",
  "term_id": "GO:0030335",
  "term_label": "positive regulation of cell migration",
  "gene_symbol": "CXCL12",
  "gene_name": "Stromal cell-derived factor 1"
}